{
  "gene": "UniProtKB:Q8IYX7",
  "term_label": "cytoskeleton",
  "gene_name": "Stabilizer of axonemal microtubules 1",
  "gene_symbol": "SAXO1",
  "term_id": "GO:0005856"
}